{
  "term_id": "GO:0035556",
  "gene_symbol": "MASTL",
  "term_label": "intracellular signal transduction",
  "gene_name": "Serine_threonine-protein kinase greatwall",
  "gene": "UniProtKB:Q96GX5"
}